{
  "term_label": "pexophagy",
  "gene_name": "Phosphatidylinositol 3-kinase catalytic subunit type 3",
  "gene": "UniProtKB:Q8NEB9",
  "gene_symbol": "PIK3C3",
  "term_id": "GO:0000425"
}